{
  "gene_name": "Enkurin",
  "term_id": "UNKNOWN:0002",
  "gene_symbol": "ENKUR",
  "term_label": "Unknown biological process",
  "gene": "UniProtKB:Q8TC29"
}